{
  "gene": "UniProtKB:P32121",
  "gene_name": "Beta-arrestin-2",
  "gene_symbol": "ARRB2",
  "term_id": "GO:0019233",
  "term_label": "sensory perception of pain"
}